{
  "gene_symbol": "TRMU",
  "gene": "UniProtKB:O75648",
  "term_label": "Unknown molecular function",
  "term_id": "UNKNOWN:0001",
  "gene_name": "Mitochondrial tRNA-specific 2-thiouridylase 1"
}